{
  "term_id": "UNKNOWN:0003",
  "gene_symbol": "ST8SIA6",
  "gene": "UniProtKB:P61647",
  "gene_name": "Alpha-2,8-sialyltransferase 8F",
  "term_label": "Unknown cellular component"
}